{
  "gene_symbol": "LOC122513141",
  "term_id": "GO:0070059",
  "term_label": "intrinsic apoptotic signaling pathway in response to endoplasmic reticulum stress",
  "gene_name": "RING-type domain-containing protein",
  "gene": "UniProtKB:A0A2R8Y4M4"
}